negative regulation of NK T cell differentiation [GO:0051137] (biological process) References: PMID:12154375, PMID:9133426 Sources: ISBN:0781735149 Definition: Any process that stops, prevents, or reduces the frequency, rate or extent of natural killer T cell differentiation. Note: Note that immunologists typically use the word 'development' to refer to cells of B or T cell lineages undergoing the process that GO describes as 'cell differentiation'. Also known as: down regulation of NK T cell differentiation, down-regulation of NK T cell differentiation, downregulation of NK T cell differentiation, negative regulation of NK T lymphocyte differentiation, negative regulation of NK T-cell differentiation, negative regulation of NK T-lymphocyte differentiation, negative regulation of NKT cell differentiation, negative regulation of NT cell differentiation, negative regulation of natural T cell differentiation, negative regulation of natural killer T cell differentiation, inhibition of NK T cell differentiation, negative regulation of NK T cell development Relationships: is a type of negative regulation of alpha-beta T cell differentiation [GO:0046639]; is a type of regulation of NK T cell differentiation [GO:0051136]; RO_0002212 NK T cell differentiation [GO:0001865]